{
  "gene": "UniProtKB:P11487",
  "term_label": "positive regulation of cell population proliferation",
  "term_id": "GO:0008284",
  "gene_symbol": "FGF3",
  "gene_name": "Fibroblast growth factor 3"
}